{
  "gene": "UniProtKB:Q5T011",
  "gene_name": "KICSTOR complex protein SZT2",
  "term_id": "UNKNOWN:0001",
  "term_label": "Unknown molecular function",
  "gene_symbol": "SZT2"
}